cyclic GMP-AMP binding [GO:0140702] (molecular function) Subtypes: GO:0061507, GO:0140703 Definition: Binding to cyclic GMP-AMP (cGAMP) nucleotide. References: PMID:23258412 Relationships: is a type of cyclic nucleotide binding [GO:0030551]